phosphoadenylylsulfatase activity [GO:0050186] (molecular function) Relationships: is a type of GO:0016819 Sources: EC:3.6.2.2 Definition: Catalysis of the reaction: 3'-phosphoadenosine 5'-phosphosulfate + H2O = adenosine 3',5'-bisphosphate + sulfate. Also known as: phosphoadenylylsulphatase activity, 3'-phosphoadenylylsulfate sulfohydrolase activity, 3-phosphoadenosine 5-phosphosulfate sulfatase activity, 3-phosphoadenylyl sulfatase activity, PAPS sulfatase activity